{
  "term_label": "Unknown cellular component",
  "gene_name": "2-methoxy-6-polyprenyl-1,4-benzoquinol methylase, mitochondrial",
  "gene": "UniProtKB:Q5HYK3",
  "gene_symbol": "COQ5",
  "term_id": "UNKNOWN:0003"
}